{
  "term_label": "extracellular space",
  "term_id": "GO:0005615",
  "gene_symbol": "HGF",
  "gene": "UniProtKB:P14210",
  "gene_name": "Hepatocyte growth factor"
}